{
  "gene": "UniProtKB:O96024",
  "term_label": "Unknown biological process",
  "gene_name": "Beta-1,3-galactosyltransferase 4",
  "gene_symbol": "B3GALT4",
  "term_id": "UNKNOWN:0002"
}